regulation of establishment or maintenance of bipolar cell polarity regulating cell shape [GO:2000100] (biological process) Definition: Any process that modulates the frequency, rate or extent of establishment or maintenance of bipolar cell polarity regulating cell shape. Relationships: is a type of regulation of establishment or maintenance of bipolar cell polarity [GO:2000099]; is a type of GO:2000769; regulates establishment or maintenance of bipolar cell polarity regulating cell shape [GO:0061246] Subtypes: regulation of establishment of bipolar cell polarity regulating cell shape [GO:0061160], GO:2000115, positive regulation of establishment or maintenance of bipolar cell polarity regulating cell shape [GO:2000247], negative regulation of establishment or maintenance of bipolar cell polarity regulating cell shape [GO:2000750] Sources: GOC:obol